{
  "term_label": "mitochondrion",
  "gene": "UniProtKB:Q3SXM5",
  "gene_name": "Inactive hydroxysteroid dehydrogenase-like protein 1",
  "term_id": "GO:0005739",
  "gene_symbol": "HSDL1"
}